D-methionine transmembrane transport [GO:0048473] (BP) Definition: The process in which D-methionine is transported across a lipid bilayer, from one side of a membrane to the other. References: PMID:12169620 Sources: GOC:mlg Relationships: is a type of amino acid transmembrane transport [GO:0003333]; is a type of methionine transport [GO:0015821]; is a type of D-amino acid transport [GO:0042940]; is a type of carboxylic acid transmembrane transport [GO:1905039]